{
  "gene": "UniProtKB:P60372",
  "gene_symbol": "KRTAP10-4",
  "term_label": "Unknown molecular function",
  "gene_name": "Keratin-associated protein 10-4",
  "term_id": "UNKNOWN:0001"
}